ribosomal small subunit binding [GO:0043024] (molecular function) Definition: Binding to a small ribosomal subunit. Sources: GOC:go_curators Relationships: is a type of ribosome binding [GO:0043022]